{
  "gene_name": "Zinc finger protein 43",
  "term_label": "regulation of transcription by RNA polymerase II",
  "gene": "UniProtKB:P17038",
  "term_id": "GO:0006357",
  "gene_symbol": "ZNF43"
}